positive regulation of translational initiation in response to starvation [GO:0071264] (biological process) Also known as: positive regulation of translational initiation in response to nutrient starvation, up regulation of translation initiation in response to starvation, up-regulation of translation initiation in response to starvation, upregulation of translation initiation in response to starvation, activation of translation initiation in response to starvation, stimulation of translation initiation in response to starvation Definition: Any process that activates or increases the frequency, rate or extent of translation initiation, as a result of deprivation of nourishment. Sources: GOC:mah Relationships: is a type of positive regulation of translation in response to stress [GO:0032056]; is a type of positive regulation of translational initiation in response to stress [GO:0032058]; is a type of regulation of translational initiation in response to starvation [GO:0071262]